{
  "term_label": "Unknown molecular function",
  "term_id": "UNKNOWN:0001",
  "gene": "UniProtKB:O14681",
  "gene_symbol": "EI24",
  "gene_name": "Etoposide-induced protein 2.4 homolog"
}